{
  "term_label": "Unknown molecular function",
  "gene": "UniProtKB:Q8TES7",
  "term_id": "UNKNOWN:0001",
  "gene_name": "Fas-binding factor 1",
  "gene_symbol": "FBF1"
}